{
  "gene_symbol": "SGTB",
  "term_id": "GO:0072380",
  "term_label": "TRC complex",
  "gene": "UniProtKB:Q96EQ0",
  "gene_name": "Small glutamine-rich tetratricopeptide repeat-containing protein beta"
}